{
  "gene_symbol": "ZNF738",
  "term_id": "GO:0000978",
  "gene_name": "Zinc finger protein 738",
  "gene": "UniProtKB:Q8NE65",
  "term_label": "RNA polymerase II cis-regulatory region sequence-specific DNA binding"
}